{
  "gene": "UniProtKB:P20339",
  "gene_name": "Ras-related protein Rab-5A",
  "term_label": "synaptic vesicle membrane",
  "gene_symbol": "RAB5A",
  "term_id": "GO:0030672"
}